trophectodermal cell fate commitment [GO:0001830] (biological process) Note: See also the Anatomical Dictionary for Mouse Development ontology terms 'TS4, trophectoderm ; EMAP:19'. Relationships: is_a cell fate commitment [GO:0045165]; is part of GO:0001829 Also known as: trophectoderm cell fate commitment Sources: GOC:dph, ISBN:0124020607, ISBN:0198542771 Definition: The cell fate commitment of precursor cells that will become trophectoderm cells.